ATPase-coupled L-glutamate tranmembrane transporter activity [GO:0102013] (molecular function) Definition: Enables the transfer of a solute or solutes from one side of a membrane to the other according to the reaction: L-glutamate(out) + ATP + H2O = L-glutamate(in) + ADP + phosphate + H+. Sources: RHEA:29035 Also known as: L-glutamate-importing ATPase activity Relationships: is a type of GO:0015426